methionine synthase activity [GO:0008705] (MF) Definition: Catalysis of the reaction: (6S)-5-methyl-5,6,7,8-tetrahydrofolate + L-homocysteine = (6S)-5,6,7,8-tetrahydrofolate + L-methionine. Also known as: 5-methyltetrahydrofolate-homocysteine S-methyltransferase activity, 5-methyltetrahydrofolate--homocysteine S-methyltransferase activity, 5-methyltetrahydrofolate--homocysteine transmethylase activity, 5-methyltetrahydrofolate:L-homocysteine S-methyltransferase activity, B12 N(5)-methyltetrahydrofolate homocysteine methyltransferase activity, B12 N5-methyltetrahydrofolate homocysteine methyltransferase activity, MetH, N(5)-methyltetrahydrofolate methyltransferase activity, N(5)-methyltetrahydrofolate--homocysteine cobalamin methyltransferase activity, N(5)-methyltetrahydrofolic--homocysteine vitamin B12 transmethylase activity, N-methyltetrahydrofolate:L-homocysteine methyltransferase activity, N5-methyltetrahydrofolate methyltransferase activity, N5-methyltetrahydrofolate-homocysteine cobalamin methyltransferase activity, N5-methyltetrahydrofolic-homocysteine vitamin B12 transmethylase activity, cobalamin-dependent methionine synthase activity, methionine synthase (cobalamin-dependent) activity, methyltetrahydrofolate--homocysteine vitamin B12 methyltransferase activity, tetrahydrofolate methyltransferase activity, tetrahydropteroylglutamate methyltransferase activity, tetrahydropteroylglutamic methyltransferase activity, vitamin B12 methyltransferase activity Relationships: is a type of GO:0008172; is a type of 5-methyltetrahydrofolate-dependent methyltransferase activity [GO:0042084]; is part of GO:0071267 Sources: EC:2.1.1.13, RHEA:11172